tripeptidase activity [GO:0034701] (molecular function) Sources: GOC:mah Subtypes: tripeptide aminopeptidase activity [GO:0045148] Definition: Catalysis of the hydrolysis of a tripeptide. Relationships: is a type of exopeptidase activity [GO:0008238]